calcium ion import into vacuole [GO:0140146] (biological process) References: PMID:8628289 Sources: GOC:vw Definition: The directed movement of calcium cations into the vacuole across the vacuolar membrane. Relationships: is a type of vacuolar transmembrane transport [GO:0034486]; is_a calcium ion transmembrane transport [GO:0070588]